{
  "gene_symbol": "PDIA2",
  "term_label": "endoplasmic reticulum",
  "gene": "UniProtKB:Q13087",
  "gene_name": "Protein disulfide-isomerase A2",
  "term_id": "GO:0005783"
}